{
  "gene_name": "WW domain-containing oxidoreductase",
  "term_id": "UNKNOWN:0001",
  "gene_symbol": "WWOX",
  "gene": "UniProtKB:Q9NZC7",
  "term_label": "Unknown molecular function"
}